{
  "gene_name": "RNA polymerase-associated protein CTR9 homolog",
  "gene_symbol": "CTR9",
  "term_id": "GO:0000993",
  "gene": "UniProtKB:Q6PD62",
  "term_label": "RNA polymerase II complex binding"
}